glomerular parietal epithelial cell fate commitment [GO:0072147] (biological process) Also known as: Bowman's capsule cell fate commitment Relationships: is_a GO:0072148; is a type of glomerular epithelial cell fate commitment [GO:0072314]; is part of glomerular parietal epithelial cell differentiation [GO:0072139] Subtypes: mesonephric glomerular parietal epithelial cell fate commitment [GO:0061255], GO:0072247 Definition: The process in which the developmental fate of a cell becomes restricted such that it will develop into a glomerular parietal epithelial cell. Glomerular parietal epithelial cells are specialized epithelial cells that form tight junctions as a barrier to protein transport. These cells may also give rise to podocytes. Sources: GOC:mtg_kidney_jan10